{
  "term_id": "UNKNOWN:0001",
  "term_label": "Unknown molecular function",
  "gene_name": "Hornerin",
  "gene_symbol": "HRNR",
  "gene": "UniProtKB:Q86YZ3"
}